{
  "term_label": "intracellular signal transduction",
  "gene": "UniProtKB:Q6NXS1",
  "gene_symbol": "PPP1R2B",
  "gene_name": "Protein phosphatase inhibitor 2 family member B",
  "term_id": "GO:0035556"
}